{
  "gene_name": "Gamma-aminobutyric acid receptor subunit gamma-2",
  "term_id": "GO:1904862",
  "term_label": "inhibitory synapse assembly",
  "gene_symbol": "GABRG2",
  "gene": "UniProtKB:P18507"
}